extraorganismal space [GO:0043245] (CC) Sources: GOC:jl Definition: The environmental space outside of an organism; this may be a host organism in the case of parasitic and symbiotic organisms. Relationships: is a type of cellular anatomical structure [GO:0110165]; is part of GO:0005576